{
  "term_label": "Unknown molecular function",
  "gene_symbol": "TMEM185B",
  "gene_name": "Transmembrane protein 185B",
  "gene": "UniProtKB:Q9H7F4",
  "term_id": "UNKNOWN:0001"
}